{
  "gene": "UniProtKB:P35212",
  "gene_name": "Gap junction alpha-4 protein",
  "term_label": "cell-cell signaling",
  "gene_symbol": "GJA4",
  "term_id": "GO:0007267"
}